{
  "gene": "UniProtKB:P56539",
  "term_label": "caveola assembly",
  "gene_symbol": "CAV3",
  "gene_name": "Caveolin-3",
  "term_id": "GO:0070836"
}